{
  "term_label": "blood coagulation",
  "term_id": "GO:0007596",
  "gene": "UniProtKB:P0CW18",
  "gene_name": "Serine protease 56",
  "gene_symbol": "PRSS56"
}